positive regulation of microglial cell migration [GO:1904141] (biological process) Also known as: up regulation of microglial cell migration, up-regulation of microglial cell migration, upregulation of microglial cell migration, activation of microglial cell migration Relationships: is a type of positive regulation of glial cell migration [GO:1903977]; is a type of GO:1904139; is a type of positive regulation of macrophage migration [GO:1905523]; positively regulates GO:1904124 Definition: Any process that activates or increases the frequency, rate or extent of microglial cell migration. References: PMID:19100238 Sources: GOC:BHF, GOC:TermGenie, GOC:nc, GO_REF:0000058